{
  "term_label": "DNA-binding transcription factor activity, RNA polymerase II-specific",
  "gene": "UniProtKB:P28358",
  "gene_symbol": "HOXD10",
  "gene_name": "Homeobox protein Hox-D10",
  "term_id": "GO:0000981"
}